proton-translocating NAD(P)+ transhydrogenase activity [GO:0008750] (molecular function) Sources: RHEA:47992 Also known as: NAD(P)+ transhydrogenase (AB-specific) activity Relationships: is a type of GO:0015078; is a type of oxidoreduction-driven active transmembrane transporter activity [GO:0015453]; is a type of active monoatomic ion transmembrane transporter activity [GO:0022853] Definition: Catalysis of the reaction: H+(in) + NAD+ + NADPH = H+(out) + NADH + NADP+.